synaptic vesicle lumen [GO:0034592] (cellular component) Definition: The volume enclosed by the synaptic vesicle membrane. Sources: GOC:rph Relationships: is a type of GO:0060205; is part of synaptic vesicle [GO:0008021]